protocadherin-alpha-v4-protocadherin-gamma-a3 complex [GO:0071185] (cellular component) Also known as: Pcdhga1-Pcdhga3 complex Definition: A protein complex that contains the cell adhesion molecules protocadherin-alpha-v4 and protocadherin-gamma-a3, and is involved in the regulation of protein localization to the plasma membrane. References: PMID:15347688 Relationships: is a type of protocadherin-alpha-protocadherin-gamma complex [GO:0071183]